{
  "term_label": "olfactory receptor activity",
  "gene": "UniProtKB:Q9H342",
  "gene_symbol": "OR51J1",
  "term_id": "GO:0004984",
  "gene_name": "Olfactory receptor 51J1"
}